negative regulation of type IV pilus biogenesis [GO:1903657] (biological process) Also known as: down regulation of TFP biogenesis, down regulation of type 4 pilus biogenesis, down regulation of type IV fimbria assembly, down regulation of type IV fimbria biogenesis, down regulation of type IV fimbriae assembly, down regulation of type IV fimbriae biogenesis, down regulation of type IV fimbrial assembly, down regulation of type IV fimbrial biogenesis, down regulation of type IV fimbrium assembly, down regulation of type IV fimbrium biogenesis, down regulation of type IV pilus biogenesis, down regulation of type IV pilus biosynthesis, down-regulation of TFP biogenesis, down-regulation of type 4 pilus biogenesis, down-regulation of type IV fimbria assembly, down-regulation of type IV fimbria biogenesis, down-regulation of type IV fimbriae assembly, down-regulation of type IV fimbriae biogenesis, down-regulation of type IV fimbrial assembly, down-regulation of type IV fimbrial biogenesis, down-regulation of type IV fimbrium assembly, down-regulation of type IV fimbrium biogenesis, down-regulation of type IV pilus biogenesis, down-regulation of type IV pilus biosynthesis, downregulation of TFP biogenesis, downregulation of type 4 pilus biogenesis, downregulation of type IV fimbria assembly, downregulation of type IV fimbria biogenesis, downregulation of type IV fimbriae assembly, downregulation of type IV fimbriae biogenesis, downregulation of type IV fimbrial assembly, downregulation of type IV fimbrial biogenesis, downregulation of type IV fimbrium assembly, downregulation of type IV fimbrium biogenesis, downregulation of type IV pilus biogenesis, downregulation of type IV pilus biosynthesis, negative regulation of TFP biogenesis, negative regulation of type 4 pilus biogenesis, negative regulation of type IV fimbria assembly, negative regulation of type IV fimbria biogenesis, negative regulation of type IV fimbriae assembly, negative regulation of type IV fimbriae biogenesis, negative regulation of type IV fimbrial assembly, negative regulation of type IV fimbrial biogenesis, negative regulation of type IV fimbrium assembly, negative regulation of type IV fimbrium biogenesis, negative regulation of type IV pilus biosynthesis, inhibition of TFP biogenesis, inhibition of type 4 pilus biogenesis, inhibition of type IV fimbria assembly, inhibition of type IV fimbria biogenesis, inhibition of type IV fimbriae assembly, inhibition of type IV fimbriae biogenesis, inhibition of type IV fimbrial assembly, inhibition of type IV fimbrial biogenesis, inhibition of type IV fimbrium assembly, inhibition of type IV fimbrium biogenesis, inhibition of type IV pilus biogenesis, inhibition of type IV pilus biosynthesis References: PMID:25049409 Sources: GOC:TermGenie, GO_REF:0000058 Relationships: is a type of GO:0031345; is a type of regulation of type IV pilus biogenesis [GO:1903656]; negatively regulates type IV pilus assembly [GO:0043683] Definition: Any process that stops, prevents or reduces the frequency, rate or extent of type IV pilus biogenesis.